D-aminoacyl-tRNA deacylase activity [GO:0051499] (molecular function) References: PMID:14527667 Sources: RHEA:13953 Definition: Catalysis of the reaction: a D-aminoacyl-tRNA + H2O = a D-alpha-amino acid + a tRNA + H+.  Removal of a D-amino acid from a charged tRNA. Relationships: is a type of GO:0002161 Subtypes: D-tyrosyl-tRNA(Tyr) deacylase activity [GO:0051500], GO:0097358